{
  "term_id": "UNKNOWN:0003",
  "term_label": "Unknown cellular component",
  "gene_name": "Immunoglobulin heavy variable 5-10-1",
  "gene": "UniProtKB:A0A0J9YXX1",
  "gene_symbol": "IGHV5-10-1"
}